{
  "term_id": "UNKNOWN:0001",
  "gene": "UniProtKB:Q9Y3A5",
  "term_label": "Unknown molecular function",
  "gene_symbol": "SBDS",
  "gene_name": "Ribosome maturation protein SBDS"
}